{
  "gene_name": "Kinesin-like protein KIF17",
  "gene": "UniProtKB:Q9P2E2",
  "term_label": "ATP hydrolysis activity",
  "gene_symbol": "KIF17",
  "term_id": "GO:0016887"
}